enkephalin processing [GO:0034230] (biological process) Relationships: is a type of peptide hormone processing [GO:0016486] Also known as: enkephalin formation, peptide enkephalin formation, peptide enkephalin processing References: PMID:8262946 Sources: GOC:BHF, GOC:mah, GOC:rl Definition: The formation of mature enkephalin, a pentapeptide hormone involved in regulating pain and nociception in the body by proteolytic processing of enkephalin propeptide.